L-histidine transmembrane export from vacuole [GO:0089708] (biological process) References: PMID:21307582 Definition: The directed movement of L-histidine out of the vacuole, across the vacuolar membrane. Relationships: is a type of amino acid transmembrane export from vacuole [GO:0032974]; is a type of GO:0089709; is a type of L-histidine transport [GO:1902024]; is a type of basic amino acid transmembrane transport [GO:1990822]